{
  "term_id": "GO:0006357",
  "gene_symbol": "FOXN1",
  "gene_name": "Forkhead box protein N1",
  "gene": "UniProtKB:O15353",
  "term_label": "regulation of transcription by RNA polymerase II"
}